{
  "gene_name": "Gamma-tubulin complex component 6",
  "term_label": "mitotic cell cycle",
  "term_id": "GO:0000278",
  "gene": "UniProtKB:Q96RT7",
  "gene_symbol": "TUBGCP6"
}